eosinophil fate specification [GO:0035857] (biological process) Relationships: is a type of cell fate specification [GO:0001708]; is part of eosinophil fate commitment [GO:0035854] Sources: CL:0000771, GOC:BHF, GOC:vk Definition: The process involved in the specification of identity of an eosinophil cell. Once specification has taken place, a cell will be committed to differentiate down a specific pathway if left in its normal environment. Also known as: eosinophil cell fate specification